{
  "term_label": "mediator complex",
  "term_id": "GO:0016592",
  "gene": "UniProtKB:Q71SY5",
  "gene_name": "Mediator of RNA polymerase II transcription subunit 25",
  "gene_symbol": "MED25"
}